{
  "gene_name": "Zinc finger MYM-type protein 4",
  "term_label": "Unknown cellular component",
  "term_id": "UNKNOWN:0003",
  "gene": "UniProtKB:Q5VZL5",
  "gene_symbol": "ZMYM4"
}